positive regulation of action potential [GO:0045760] (biological process) Relationships: is a type of positive regulation of biological process [GO:0048518]; is a type of GO:0098900; positively regulates GO:0001508 Definition: Any process that activates or increases the frequency, rate or extent of action potential creation, propagation or termination. This typically occurs via modulation of the activity or expression of voltage-gated ion channels. Subtypes: GO:1903947, positive regulation of atrial cardiac muscle cell action potential [GO:1903949], positive regulation of AV node cell action potential [GO:1903951], positive regulation of neuronal action potential [GO:1904457] Sources: GOC:go_curators Also known as: up regulation of action potential, up-regulation of action potential, upregulation of action potential, activation of action potential, stimulation of action potential